{
  "term_id": "GO:0005737",
  "gene_name": "Dynein light chain Tctex-type 3",
  "gene": "UniProtKB:P51808",
  "gene_symbol": "DYNLT3",
  "term_label": "cytoplasm"
}